{
  "term_id": "GO:0005262",
  "term_label": "calcium channel activity",
  "gene_name": "Sodium_potassium_calcium exchanger 5",
  "gene": "UniProtKB:Q71RS6",
  "gene_symbol": "SLC24A5"
}